{
  "gene_symbol": "MLNR",
  "gene_name": "Motilin receptor",
  "term_id": "GO:0007186",
  "gene": "UniProtKB:O43193",
  "term_label": "G protein-coupled receptor signaling pathway"
}